{
  "gene_name": "Tetraspanin-5",
  "gene": "UniProtKB:P62079",
  "term_id": "UNKNOWN:0001",
  "term_label": "Unknown molecular function",
  "gene_symbol": "TSPAN5"
}